{
  "gene_symbol": "TRIM65",
  "term_id": "UNKNOWN:0001",
  "gene_name": "E3 ubiquitin-protein ligase TRIM65",
  "gene": "UniProtKB:Q6PJ69",
  "term_label": "Unknown molecular function"
}